liver regeneration [GO:0097421] (biological process) Relationships: is a type of GO:0001889; is_a animal organ regeneration [GO:0031100] References: PMID:19447520 Sources: GOC:gap Definition: The regrowth of lost or destroyed liver.